{
  "gene": "UniProtKB:Q8WV92",
  "term_label": "midbody abscission",
  "gene_name": "MIT domain-containing protein 1",
  "gene_symbol": "MITD1",
  "term_id": "GO:0061952"
}